{
  "gene_name": "Rho guanine nucleotide exchange factor 7",
  "gene_symbol": "ARHGEF7",
  "gene": "UniProtKB:Q14155",
  "term_label": "lamellipodium",
  "term_id": "GO:0030027"
}